{
  "term_label": "Unknown molecular function",
  "gene": "UniProtKB:P0C7H8",
  "gene_name": "Keratin-associated protein 2-3",
  "term_id": "UNKNOWN:0001",
  "gene_symbol": "KRTAP2-3"
}